{
  "gene": "UniProtKB:Q8WUD4",
  "gene_symbol": "CCDC12",
  "term_label": "U2-type spliceosomal complex",
  "term_id": "GO:0005684",
  "gene_name": "Coiled-coil domain-containing protein 12"
}